{
  "term_label": "positive regulation of DNA replication",
  "term_id": "GO:0045740",
  "gene_name": "CST complex subunit CTC1",
  "gene": "UniProtKB:Q2NKJ3",
  "gene_symbol": "CTC1"
}